COPII vesicle uncoating [GO:0090112] (biological process) Sources: GOC:ascb_2009, GOC:dph, GOC:tb Relationships: is_a vesicle uncoating [GO:0072319]; is part of endoplasmic reticulum to Golgi vesicle-mediated transport [GO:0006888] Regulation: RO_0002211 by regulation of COPII vesicle uncoating [GO:0090111] Definition: The process in which COPII vesicle coat proteins are disassembled, and released.